{
  "gene": "UniProtKB:Q96MR7",
  "term_id": "UNKNOWN:0001",
  "term_label": "Unknown molecular function",
  "gene_symbol": "OBSCN-AS1",
  "gene_name": "Putative uncharacterized protein OBSCN-AS1"
}